{
  "term_id": "GO:0005813",
  "term_label": "centrosome",
  "gene_name": "Disrupted in schizophrenia 1 protein",
  "gene": "UniProtKB:Q9NRI5",
  "gene_symbol": "DISC1"
}